dCDP biosynthetic process [GO:0006240] (biological process) Also known as: dCDP anabolism, dCDP biosynthesis, dCDP formation, dCDP synthesis Regulation: RO_0002211 by regulation of dCDP biosynthetic process [GO:1903528]; negatively regulated by negative regulation of dCDP biosynthetic process [GO:1903529] Sources: ISBN:0198506732 Relationships: is a type of pyrimidine deoxyribonucleoside diphosphate biosynthetic process [GO:0009197]; is_a pyrimidine deoxyribonucleotide biosynthetic process [GO:0009221]; is a type of GO:0046062 Definition: The chemical reactions and pathways resulting in the formation of dCDP, deoxycytidine 5'-diphosphate.